{
  "term_id": "GO:0016493",
  "gene_name": "C-C chemokine receptor type 8",
  "term_label": "C-C chemokine receptor activity",
  "gene": "UniProtKB:P51685",
  "gene_symbol": "CCR8"
}